negative regulation of cellular hyperosmotic salinity response [GO:1900070] (biological process) Relationships: is a type of negative regulation of cellular process [GO:0048523]; is a type of regulation of cellular hyperosmotic salinity response [GO:1900069]; is a type of negative regulation of response to salt stress [GO:1901001]; negatively regulates cellular hyperosmotic salinity response [GO:0071475] Definition: Any process that stops, prevents or reduces the frequency, rate or extent of cellular hyperosmotic salinity response. Also known as: down regulation of cellular response to hyperosmotic salt stress, down-regulation of cellular response to hyperosmotic salt stress, downregulation of cellular response to hyperosmotic salt stress, negative regulation of cellular response to hyperosmotic salt stress, inhibition of cellular hyperosmotic salinity response, inhibition of cellular response to hyperosmotic salt stress, down regulation of cellular hyperosmotic salinity response, down-regulation of cellular hyperosmotic salinity response, downregulation of cellular hyperosmotic salinity response References: PMID:16278455 Sources: GOC:TermGenie, GOC:dgf